{
  "gene_symbol": "GRIN3B",
  "gene_name": "Glutamate receptor ionotropic, NMDA 3B",
  "term_label": "NMDA glutamate receptor activity",
  "term_id": "GO:0004972",
  "gene": "UniProtKB:O60391"
}